{
  "gene_symbol": "HCRTR2",
  "term_id": "GO:0032870",
  "gene_name": "Orexin receptor type 2",
  "term_label": "cellular response to hormone stimulus",
  "gene": "UniProtKB:O43614"
}